{
  "gene_name": "Regulator of nonsense transcripts 3A",
  "term_id": "GO:0042162",
  "gene": "UniProtKB:Q9H1J1",
  "term_label": "telomeric DNA binding",
  "gene_symbol": "UPF3A"
}